{
  "gene": "UniProtKB:P35321",
  "term_id": "GO:0001533",
  "term_label": "cornified envelope",
  "gene_name": "Cornifin-A",
  "gene_symbol": "SPRR1A"
}